regulation of mRNA stability [GO:0043488] (biological process) Definition: Any process that modulates the propensity of mRNA molecules to degradation. Includes processes that both stabilize and destabilize mRNAs. Sources: GOC:jl Relationships: is a type of regulation of RNA stability [GO:0043487]; is a type of GO:0061013 Subtypes: GO:0010610, regulation of mitochondrial mRNA stability [GO:0044528], mRNA stabilization [GO:0048255], mRNA destabilization [GO:0061157], regulation of nuclear-transcribed mRNA catabolic process, deadenylation-dependent decay [GO:1900151], GO:1902629, regulation of 3'-UTR-mediated mRNA stabilization [GO:1905868]